negative regulation of atrichoblast fate specification [GO:0010060] (biological process) Relationships: is a type of GO:0009996; is a type of GO:0010058; is a type of negative regulation of plant epidermal cell differentiation [GO:1903889]; negatively regulates atrichoblast fate specification [GO:0010056] Also known as: down regulation of atrichoblast fate, down-regulation of atrichoblast fate, downregulation of atrichoblast fate, inhibition of atrichoblast fate Sources: GOC:tb Definition: Any process that suppresses atrichoblast fate specification.